regulation of lysine biosynthetic process via alpha-aminoadipate and saccharopine [GO:2001194] (biological process) Definition: Any process that modulates the frequency, rate or extent of lysine biosynthetic process via alpha-aminoadipate and saccharopine. Also known as: regulation of lysine biosynthesis via aminoadipic acid and saccharopine, regulation of lysine biosynthetic process via aminoadipic acid and saccharopine Sources: GOC:obol Subtypes: negative regulation of lysine biosynthetic process via alpha-aminoadipate and saccharopine [GO:2001195], positive regulation of lysine biosynthetic process via alpha-aminoadipate and saccharopine [GO:2001196] Relationships: is a type of regulation of lysine biosynthetic process via aminoadipic acid [GO:1902986]; regulates lysine biosynthetic process via alpha-aminoadipate and saccharopine [GO:0051975]